{
  "gene_name": "Probable inactive serine protease 37",
  "gene": "UniProtKB:A4D1T9",
  "term_id": "GO:0001669",
  "gene_symbol": "PRSS37",
  "term_label": "acrosomal vesicle"
}